{
  "gene_symbol": "PM20D2",
  "term_id": "UNKNOWN:0002",
  "term_label": "Unknown biological process",
  "gene": "UniProtKB:Q8IYS1",
  "gene_name": "Xaa-Arg dipeptidase"
}